{
  "term_id": "GO:0007088",
  "gene_name": "Protein aurora borealis",
  "term_label": "regulation of mitotic nuclear division",
  "gene": "UniProtKB:Q6PGQ7",
  "gene_symbol": "BORA"
}